IkappaB kinase complex binding [GO:0106137] (molecular function) Relationships: is a type of GO:0044877 References: PMID:12492477 Sources: GOC:pga Definition: Binding to a IkappaB kinase complex.